cysteine biosynthetic process [GO:0019344] (biological process) Also known as: cysteine anabolism, cysteine biosynthesis, cysteine formation, cysteine synthesis Sources: GOC:go_curators Relationships: is_a sulfur amino acid biosynthetic process [GO:0000097]; is_a cysteine metabolic process [GO:0006534]; is a type of serine family amino acid biosynthetic process [GO:0009070] Subtypes: cysteine biosynthetic process from serine [GO:0006535], cysteine biosynthetic process via cystathionine [GO:0019343], cysteine biosynthetic process via S-sulfo-L-cysteine [GO:0019345] Definition: The chemical reactions and pathways resulting in the formation of cysteine, 2-amino-3-mercaptopropanoic acid.